{
  "gene_symbol": "MX1",
  "gene": "UniProtKB:P20591",
  "gene_name": "Interferon-induced GTP-binding protein Mx1",
  "term_label": "cytoplasm",
  "term_id": "GO:0005737"
}